negative regulation of chemokinesis [GO:1904366] (biological process) Relationships: is_a GO:0032102; is a type of GO:1904365; negatively regulates chemokinesis [GO:0042466] Also known as: down regulation of chemokinesis, down-regulation of chemokinesis, downregulation of chemokinesis, inhibition of chemokinesis References: PMID:8679543 Sources: GOC:TermGenie, GO_REF:0000058 Definition: Any process that stops, prevents or reduces the frequency, rate or extent of chemokinesis.